{
  "gene": "UniProtKB:Q9H4F8",
  "term_label": "extracellular matrix binding",
  "gene_name": "SPARC-related modular calcium-binding protein 1",
  "gene_symbol": "SMOC1",
  "term_id": "GO:0050840"
}